{
  "term_id": "GO:0043066",
  "gene_symbol": "HGF",
  "gene": "UniProtKB:P14210",
  "gene_name": "Hepatocyte growth factor",
  "term_label": "negative regulation of apoptotic process"
}